{
  "gene": "UniProtKB:Q13572",
  "term_id": "GO:0047325",
  "term_label": "inositol-3,4,5,6-tetrakisphosphate 1-kinase activity",
  "gene_name": "Inositol-tetrakisphosphate 1-kinase",
  "gene_symbol": "ITPK1"
}